{
  "term_label": "Unknown biological process",
  "gene_name": "Coiled-coil domain-containing protein 150",
  "gene_symbol": "CCDC150",
  "gene": "UniProtKB:Q8NCX0",
  "term_id": "UNKNOWN:0002"
}